{
  "gene_symbol": "SLC6A19",
  "gene": "UniProtKB:Q695T7",
  "gene_name": "Sodium-dependent neutral amino acid transporter B(0)AT1",
  "term_id": "GO:0031526",
  "term_label": "brush border membrane"
}